{
  "term_id": "GO:0000978",
  "gene": "UniProtKB:Q9HBT8",
  "gene_name": "Zinc finger protein 286A",
  "term_label": "RNA polymerase II cis-regulatory region sequence-specific DNA binding",
  "gene_symbol": "ZNF286A"
}